{
  "gene": "UniProtKB:Q8N1T3",
  "term_label": "cytoplasm",
  "gene_symbol": "MYO1H",
  "term_id": "GO:0005737",
  "gene_name": "Unconventional myosin-Ih"
}